formation of stylet for nutrient acquisition [GO:0085001] (biological process) Relationships: is a type of formation of specialized structure for nutrient acquisition [GO:0052093] Also known as: formation by symbiont of stylet for nutrient acquisition from host Definition: The assembly of a stylet, a hollow protrusible spear-like symbiont structure projected into the host cell for the purpose of obtaining nutrients. The host is defined as the larger of the organisms involved in a symbiotic interaction. Sources: GOC:pamgo_curators